{
  "gene": "UniProtKB:P35498",
  "gene_name": "Sodium channel protein type 1 subunit alpha",
  "term_id": "GO:0005248",
  "term_label": "voltage-gated sodium channel activity",
  "gene_symbol": "SCN1A"
}